{
  "term_label": "protein localization to plasma membrane",
  "gene_name": "Na(+)_H(+) exchange regulatory cofactor NHE-RF2",
  "gene_symbol": "NHERF2",
  "gene": "UniProtKB:Q15599",
  "term_id": "GO:0072659"
}